{
  "term_id": "GO:0006457",
  "gene_symbol": "DNAJB4",
  "gene_name": "DnaJ homolog subfamily B member 4",
  "term_label": "protein folding",
  "gene": "UniProtKB:Q9UDY4"
}